calcium activated phospholipid scrambling [GO:0061588] (biological process) References: PMID:23532839 Sources: GOC:krc Relationships: is a type of plasma membrane phospholipid scrambling [GO:0017121] Definition: The movement of a population of phospholipid molecules from one leaflet of the plasma membrane bilayer to the opposite leaflet as a result of a calcium stimulus. Subtypes: calcium activated phosphatidylserine scrambling [GO:0061589], calcium activated phosphatidylcholine scrambling [GO:0061590], calcium activated galactosylceramide scrambling [GO:0061591]